{
  "gene_name": "Large ribosomal subunit protein uL2",
  "gene": "UniProtKB:P62917",
  "term_id": "GO:0002181",
  "term_label": "cytoplasmic translation",
  "gene_symbol": "RPL8"
}